glutamine binding [GO:0070406] (molecular function) Sources: CHEBI:28300, GOC:ecd Definition: Binding to glutamine, 2,5-diamino-5-oxopentanoic acid. Relationships: is a type of GO:0031406